histone modifying activity [GO:0140993] (molecular function) Definition: A catalytic activity that acts on a histone protein. Reversible histone modifications contribute to regulation of gene expression. Sources: GOC:pg Relationships: is_a catalytic activity, acting on a protein [GO:0140096]; is part of chromatin remodeling [GO:0006338] Subtypes: histone acetyltransferase activity [GO:0004402], histone deacetylase activity [GO:0004407], histone demethylase activity [GO:0032452], histone kinase activity [GO:0035173], histone methyltransferase activity [GO:0042054], histone propionyltransferase activity [GO:0061922], histone succinyltransferase activity [GO:0106078], histone glutaryltransferase activity [GO:0106229], histone serotonyltransferase activity [GO:0120295], histone dopaminyltransferase activity [GO:0120297], GO:0120301, histone crotonyltransferase activity [GO:0140068], histone butyryltransferase activity [GO:0140069], GO:0140218, histone methacryllysine demethacrylase activity [GO:0140219], histone benzoyllysine debenzoylase activity [GO:0140228], histone isonicotinyllysine deisonicotinylase activity [GO:0140229], histone isonicotinyltransferase activity [GO:0140230], histone phosphatase activity [GO:0140789], histone arginine deiminase activity [GO:0140794], histone ubiquitin ligase activity [GO:0140852], GO:0140934, GO:0160009